{
  "gene_name": "Ribosome production factor 2 homolog",
  "gene": "UniProtKB:Q9H7B2",
  "term_id": "GO:0019843",
  "gene_symbol": "RPF2",
  "term_label": "rRNA binding"
}